{
  "gene_name": "Platelet glycoprotein VI",
  "term_label": "transmembrane signaling receptor activity",
  "term_id": "GO:0004888",
  "gene": "UniProtKB:Q9HCN6",
  "gene_symbol": "GP6"
}